{
  "term_id": "GO:0007189",
  "gene_name": "Adhesion G protein-coupled receptor F4",
  "gene": "UniProtKB:Q8IZF3",
  "gene_symbol": "ADGRF4",
  "term_label": "adenylate cyclase-activating G protein-coupled receptor signaling pathway"
}